{
  "term_label": "trans-synaptic signaling, modulating synaptic transmission",
  "gene_name": "Cerebellin-4",
  "term_id": "GO:0099550",
  "gene_symbol": "CBLN4",
  "gene": "UniProtKB:Q9NTU7"
}